mitochondrial RNA metabolic process [GO:0000959] (biological process) Definition: The chemical reactions and pathways involving RNA transcribed from the mitochondrial genome and occurring in the mitochondrion. Subtypes: mitochondrial RNA catabolic process [GO:0000957], mitochondrial transcription [GO:0006390], transcription initiation at mitochondrial promoter [GO:0006391], transcription elongation by mitochondrial RNA polymerase [GO:0006392], GO:0006393, tRNA aminoacylation for mitochondrial protein translation [GO:0070127], GO:0090615, mitochondrial tRNA processing [GO:0090646], mitochondrial RNA modification [GO:1900864] Sources: GOC:krc, GOC:mah Relationships: is a type of RNA metabolic process [GO:0016070]; occurs in mitochondrion [GO:0005739]